{
  "gene_symbol": "PAFAH1B1",
  "term_id": "GO:0007281",
  "gene": "UniProtKB:P43034",
  "gene_name": "Platelet-activating factor acetylhydrolase IB subunit beta",
  "term_label": "germ cell development"
}